{
  "gene": "UniProtKB:Q86WN2",
  "gene_name": "Interferon epsilon",
  "term_id": "GO:0005125",
  "gene_symbol": "IFNE",
  "term_label": "cytokine activity"
}